{
  "gene": "UniProtKB:Q8NGG4",
  "gene_symbol": "OR8H1",
  "term_label": "sensory perception of smell",
  "gene_name": "Olfactory receptor 8H1",
  "term_id": "GO:0007608"
}